{
  "term_id": "GO:0006122",
  "gene_symbol": "UQCR10",
  "term_label": "mitochondrial electron transport, ubiquinol to cytochrome c",
  "gene_name": "Cytochrome b-c1 complex subunit 9",
  "gene": "UniProtKB:Q9UDW1"
}